{
  "gene_name": "Cytoplasmic phosphatidylinositol transfer protein 1",
  "gene_symbol": "PITPNC1",
  "term_label": "phosphatidylinositol transfer activity",
  "gene": "UniProtKB:Q9UKF7",
  "term_id": "GO:0008526"
}